{
  "term_label": "Unknown molecular function",
  "term_id": "UNKNOWN:0001",
  "gene_name": "Immunoglobulin lambda variable 4-3",
  "gene": "UniProtKB:A0A075B6K6",
  "gene_symbol": "IGLV4-3"
}